{
  "gene_symbol": "FOXM1",
  "gene_name": "Forkhead box protein M1",
  "gene": "UniProtKB:Q08050",
  "term_id": "GO:0007346",
  "term_label": "regulation of mitotic cell cycle"
}